proton-transporting V-type ATPase complex [GO:0033176] (CC) Relationships: is_a proton-transporting two-sector ATPase complex [GO:0016469]; is_a GO:0090533; is_a ATPase complex [GO:1904949] Also known as: hydrogen-translocating V-type ATPase complex References: PMID:16449553 Sources: GOC:mah, ISBN:0716743663 Subtypes: GO:0016471, GO:0033181 Definition: A proton-transporting two-sector ATPase complex that couples ATP hydrolysis to the transport of protons across a concentration gradient. The resulting transmembrane electrochemical potential of H+ is used to drive a variety of (i) secondary active transport systems via H+-dependent symporters and antiporters and (ii) channel-mediated transport systems. The complex comprises a membrane sector (V0) that carries out proton transport and a cytoplasmic compartment sector (V1) that catalyzes ATP hydrolysis. V-type ATPases are found in the membranes of organelles such as vacuoles, endosomes, and lysosomes, and in the plasma membrane.